{
  "gene_symbol": "CLIP1",
  "gene_name": "CAP-Gly domain-containing linker protein 1",
  "term_label": "cytoplasmic microtubule organization",
  "gene": "UniProtKB:P30622",
  "term_id": "GO:0031122"
}